{
  "gene": "UniProtKB:A4D161",
  "term_label": "Unknown biological process",
  "gene_name": "Protein FAM221A",
  "gene_symbol": "FAM221A",
  "term_id": "UNKNOWN:0002"
}